positive phototaxis [GO:0046956] (biological process) Also known as: positive phototactic behavior, positive phototactic behaviour, positive taxis in response to light Relationships: is a type of phototaxis [GO:0042331]; is a type of positive energy taxis [GO:0052128] Definition: The directed movement of a cell or organism towards a source of light. Sources: GOC:ai